endocardial cushion cell fate determination [GO:0061446] (biological process) Relationships: is a type of cardiac cell fate determination [GO:0060913]; is part of endocardial cushion cell fate commitment [GO:0061445] Sources: GOC:BHF, GOC:dph Definition: The process involved in endocardial cushion cell fate commitment. Once determination has taken place, a cell becomes committed to differentiate down a particular pathway regardless of its environment.